{
  "gene_name": "Oligodendrocyte-myelin glycoprotein",
  "gene": "UniProtKB:P23515",
  "term_id": "UNKNOWN:0001",
  "term_label": "Unknown molecular function",
  "gene_symbol": "OMG"
}